3-carboxyethylcatechol 2,3-dioxygenase activity [GO:0047070] (molecular function) Sources: EC:1.13.11.16, MetaCyc:1.13.11.16-RXN Also known as: 2,3-dihydroxy-beta-phenylpropionate oxygenase activity, 2,3-dihydroxy-beta-phenylpropionic dioxygenase activity, 3-(2,3-dihydroxyphenyl)propanoate:oxygen 1,2-oxidoreductase (decyclizing), 3-(2,3-dihydroxyphenyl)propanoate:oxygen 1,2-oxidoreductase activity Definition: Catalysis of the reaction: O2 + 3-(2,3-dihydroxyphenyl)propanoate = 2-hydroxy-6-oxonona-2,4-diene-1,9-dioate. Relationships: is a type of oxidoreductase activity, acting on single donors with incorporation of molecular oxygen, incorporation of two atoms of oxygen [GO:0016702]